negative regulation of flower development [GO:0009910] (biological process) Sources: GOC:go_curators Also known as: down regulation of flower development, down-regulation of flower development, downregulation of flower development, inhibition of flower development Relationships: is a type of GO:0009909; is a type of negative regulation of post-embryonic development [GO:0048581]; is a type of negative regulation of reproductive process [GO:2000242]; RO_0002212 GO:0009908 Definition: Any process that stops, prevents, or reduces the frequency, rate or extent of flower development.